{
  "term_id": "GO:0048874",
  "term_label": "host-mediated modulation of intestinal microbiota composition",
  "gene_name": "Alpha-N-acetylgalactosaminide alpha-2,6-sialyltransferase 1",
  "gene_symbol": "ST6GALNAC1",
  "gene": "UniProtKB:Q9NSC7"
}